{
  "term_label": "chromatin remodeling",
  "gene_name": "Bromodomain-containing protein 4",
  "gene_symbol": "BRD4",
  "gene": "UniProtKB:O60885",
  "term_id": "GO:0006338"
}